{
  "gene": "UniProtKB:Q12965",
  "gene_name": "Unconventional myosin-Ie",
  "gene_symbol": "MYO1E",
  "term_label": "plasma membrane",
  "term_id": "GO:0005886"
}